maintenance of protease location in T cell secretory granule [GO:0033379] (biological process) Subtypes: maintenance of granzyme B location in T cell secretory granule [GO:0033382] Sources: GOC:dph, GOC:mah, GOC:tb Also known as: maintenance of protease localization in T lymphocyte secretory granule, maintenance of protease localization in T-cell secretory granule, maintenance of protease localization in T-lymphocyte secretory granule, maintenance of protease localization in T cell secretory granule Definition: A process in which a protease is maintained in a secretory granule in a T cell and prevented from moving elsewhere. Relationships: is a type of maintenance of protein location in T cell secretory granule [GO:0033377]; is part of GO:0033375